{
  "gene_name": "Zinc finger protein 93",
  "term_id": "GO:0000981",
  "term_label": "DNA-binding transcription factor activity, RNA polymerase II-specific",
  "gene": "UniProtKB:P35789",
  "gene_symbol": "ZNF93"
}